{
  "term_label": "ubiquitin-like ligase-substrate adaptor activity",
  "gene": "UniProtKB:Q9Y297",
  "gene_symbol": "BTRC",
  "term_id": "GO:1990756",
  "gene_name": "F-box_WD repeat-containing protein 1A"
}